{
  "term_label": "peptide hormone processing",
  "gene_symbol": "FURIN",
  "gene": "UniProtKB:P09958",
  "term_id": "GO:0016486",
  "gene_name": "Furin"
}